{
  "term_id": "GO:0060090",
  "gene": "UniProtKB:O14490",
  "gene_name": "Disks large-associated protein 1",
  "term_label": "molecular adaptor activity",
  "gene_symbol": "DLGAP1"
}